{
  "term_id": "GO:0000124",
  "gene_symbol": "TADA1",
  "gene_name": "Transcriptional adapter 1",
  "term_label": "SAGA complex",
  "gene": "UniProtKB:Q96BN2"
}